{
  "term_id": "GO:0005886",
  "gene_name": "Prostaglandin F2-alpha receptor",
  "gene": "UniProtKB:P43088",
  "term_label": "plasma membrane",
  "gene_symbol": "PTGFR"
}